negative regulation of Rac protein signal transduction [GO:0035021] (biological process) Definition: Any process that stops, prevents, or reduces the frequency, rate or extent of Rac protein signal transduction. Sources: GOC:bf Also known as: down regulation of Rac protein signal transduction, down-regulation of Rac protein signal transduction, downregulation of Rac protein signal transduction, inhibition of Rac protein signal transduction Relationships: is a type of regulation of Rac protein signal transduction [GO:0035020]; is_a negative regulation of small GTPase mediated signal transduction [GO:0051058]; negatively regulates GO:0016601